{
  "term_label": "Golgi apparatus",
  "gene": "UniProtKB:Q9ULW5",
  "term_id": "GO:0005794",
  "gene_name": "Ras-related protein Rab-26",
  "gene_symbol": "RAB26"
}